biopterin transport [GO:0015877] (biological process) Relationships: is a type of nitrogen compound transport [GO:0071705] Definition: The directed movement of biopterin into, out of or within a cell, or between cells, by means of some agent such as a transporter or pore. Biopterin is a growth factor for certain protozoans and some insects; it is widely distributed in tissues and functions in a reduced form, tetrahydrobiopterin, as a hydroxylation coenzyme. Sources: GOC:ai